recycling endosome lumen [GO:0034777] (cellular component) Sources: GOC:rph Definition: The volume enclosed by the membranes of a recycling endosome. Relationships: is a type of endosome lumen [GO:0031904]; is part of GO:0055037